{
  "term_label": "Unknown biological process",
  "term_id": "UNKNOWN:0002",
  "gene": "UniProtKB:P24311",
  "gene_name": "Cytochrome c oxidase subunit 7B, mitochondrial",
  "gene_symbol": "COX7B"
}